{
  "gene_symbol": "ADGRB3",
  "term_label": "postsynapse",
  "term_id": "GO:0098794",
  "gene": "UniProtKB:O60242",
  "gene_name": "Adhesion G protein-coupled receptor B3"
}